{
  "gene_name": "Short transient receptor potential channel 6",
  "gene": "UniProtKB:Q9Y210",
  "term_id": "GO:0007338",
  "gene_symbol": "TRPC6",
  "term_label": "single fertilization"
}